{
  "term_label": "cytokine binding",
  "term_id": "GO:0019955",
  "gene_symbol": "OSMR",
  "gene_name": "Oncostatin-M-specific receptor subunit beta",
  "gene": "UniProtKB:Q99650"
}